{
  "term_id": "GO:0000977",
  "gene_symbol": "ZFP37",
  "term_label": "RNA polymerase II transcription regulatory region sequence-specific DNA binding",
  "gene": "UniProtKB:Q9Y6Q3",
  "gene_name": "Zinc finger protein 37 homolog"
}